negative regulation of T-helper 1 type immune response [GO:0002826] (biological process) Sources: GOC:add Subtypes: negative regulation of T-helper 1 cell differentiation [GO:0045626], GO:2000555 Also known as: down regulation of T-helper 1 type immune response, down-regulation of T-helper 1 type immune response, downregulation of T-helper 1 type immune response, inhibition of T-helper 1 type immune response Relationships: is a type of negative regulation of adaptive immune response based on somatic recombination of immune receptors built from immunoglobulin superfamily domains [GO:0002823]; is_a regulation of T-helper 1 type immune response [GO:0002825]; RO_0002212 T-helper 1 type immune response [GO:0042088] Definition: Any process that stops, prevents, or reduces the frequency, rate, or extent of a T-helper 1 type immune response.